glial cell-derived neurotrophic factor receptor binding [GO:0030116] (molecular function) Also known as: glial cell line-derived neurotrophic factor receptor ligand, glial cell line-derived neurotrophic factor receptor binding Relationships: is a type of growth factor receptor binding [GO:0070851] References: PMID:11476867 Sources: GOC:vw Definition: A growth factor that binds selectively and non-covalently to glial cell-derived neurotrophic factor receptors.